{
  "gene_name": "Small lysine-rich protein 1",
  "term_label": "Unknown biological process",
  "term_id": "UNKNOWN:0002",
  "gene_symbol": "SMKR1",
  "gene": "UniProtKB:H3BMG3"
}